{
  "gene": "UniProtKB:Q8WXH2",
  "term_id": "GO:0030314",
  "gene_symbol": "JPH3",
  "gene_name": "Junctophilin-3",
  "term_label": "junctional membrane complex"
}